{
  "term_id": "GO:0005794",
  "gene_name": "Putative glycosyltransferase 6 domain-containing protein 1",
  "term_label": "Golgi apparatus",
  "gene_symbol": "GLT6D1",
  "gene": "UniProtKB:Q7Z4J2"
}